plasma lipoprotein particle oxidation [GO:0034441] (biological process) Sources: GOC:BHF, GOC:mah Regulation: regulated by regulation of plasma lipoprotein oxidation [GO:0034444]; negatively regulated by GO:0034445 Definition: The modification of a lipid or protein within a plasma lipoprotein particle by oxidation of the lipid or one or more amino acids. Relationships: is a type of GO:0034369 Also known as: plasma lipoprotein oxidation